{
  "term_label": "mRNA binding",
  "term_id": "GO:0003729",
  "gene_symbol": "DDX21",
  "gene_name": "Nucleolar RNA helicase 2",
  "gene": "UniProtKB:Q9NR30"
}